{
  "term_label": "synaptic transmission, GABAergic",
  "gene_name": "Gamma-aminobutyric acid receptor subunit beta-1",
  "term_id": "GO:0051932",
  "gene_symbol": "GABRB1",
  "gene": "UniProtKB:P18505"
}